{
  "gene_symbol": "PCBP2",
  "term_label": "single-stranded DNA binding",
  "gene_name": "Poly(rC)-binding protein 2",
  "gene": "UniProtKB:Q15366",
  "term_id": "GO:0003697"
}